{
  "term_label": "Unknown biological process",
  "gene": "UniProtKB:Q3MIP1",
  "term_id": "UNKNOWN:0002",
  "gene_name": "Inositol 1,4,5-trisphosphate receptor-interacting protein-like 2",
  "gene_symbol": "ITPRIPL2"
}